positive regulation of engulfment of apoptotic cell [GO:1901076] (biological process) Relationships: is a type of positive regulation of phagocytosis, engulfment [GO:0060100]; is a type of GO:1901074; is_a positive regulation of apoptotic cell clearance [GO:2000427]; positively regulates engulfment of apoptotic cell [GO:0043652] Definition: Any process that activates or increases the frequency, rate or extent of engulfment of apoptotic cell. References: PMID:19402756 Sources: GO:kmv, GOC:TermGenie Also known as: positive regulation of engulfment of apoptotic cell corpse, positive regulation of engulfment of cell corpse, up regulation of engulfment of apoptotic cell, up regulation of engulfment of apoptotic cell corpse, up regulation of engulfment of cell corpse, up-regulation of engulfment of apoptotic cell, up-regulation of engulfment of apoptotic cell corpse, up-regulation of engulfment of cell corpse, upregulation of engulfment of apoptotic cell, upregulation of engulfment of apoptotic cell corpse, upregulation of engulfment of cell corpse, activation of engulfment of apoptotic cell, activation of engulfment of apoptotic cell corpse, activation of engulfment of cell corpse